low voltage-gated calcium channel activity [GO:0008332] (molecular function) References: PMID:16382099 Sources: GOC:mtg_transport, ISBN:0815340729 Relationships: is a type of voltage-gated calcium channel activity [GO:0005245] Also known as: low voltage gated calcium channel activity, low voltage-dependent calcium channel activity, T-type calcium channel Definition: Enables the transmembrane transfer of a calcium ion by a low voltage-gated channel. A low voltage-gated channel is a channel whose open state is dependent on low voltage across the membrane in which it is embedded.